{
  "gene_name": "HAUS augmin-like complex subunit 2",
  "gene_symbol": "HAUS2",
  "gene": "UniProtKB:Q9NVX0",
  "term_label": "mitotic spindle microtubule",
  "term_id": "GO:1990498"
}